{
  "term_label": "serine-type endopeptidase activity",
  "gene_name": "Myeloblastin",
  "gene": "UniProtKB:P24158",
  "term_id": "GO:0004252",
  "gene_symbol": "PRTN3"
}